{
  "gene": "UniProtKB:Q8N565",
  "term_label": "melanocyte differentiation",
  "gene_symbol": "MREG",
  "gene_name": "Melanoregulin",
  "term_id": "GO:0030318"
}